{
  "term_id": "GO:0030198",
  "gene_name": "Collagen alpha-1(VII) chain",
  "term_label": "extracellular matrix organization",
  "gene": "UniProtKB:Q02388",
  "gene_symbol": "COL7A1"
}